parathyroid hormone receptor activity [GO:0004991] (MF) Definition: Combining with parathyroid hormone to initiate a change in cell activity. Relationships: is a type of G protein-coupled receptor activity [GO:0004930] Sources: GOC:mah